{
  "term_label": "5'-nucleotidase activity",
  "gene_name": "Cytosolic purine 5'-nucleotidase",
  "gene_symbol": "NT5C2",
  "term_id": "GO:0008253",
  "gene": "UniProtKB:P49902"
}